{
  "gene": "UniProtKB:P37023",
  "term_id": "GO:0009953",
  "gene_symbol": "ACVRL1",
  "gene_name": "Serine_threonine-protein kinase receptor R3",
  "term_label": "dorsal/ventral pattern formation"
}